{
  "gene_symbol": "PIERCE2",
  "gene": "UniProtKB:H3BRN8",
  "term_label": "Unknown cellular component",
  "term_id": "UNKNOWN:0003",
  "gene_name": "Piercer of microtubule wall 2 protein"
}